negative regulation of endocytic recycling [GO:2001136] (biological process) Sources: GOC:obol Subtypes: negative regulation of endosome to plasma membrane protein transport [GO:1905750] Also known as: negative regulation of retrograde transport of endocytic vesicles Definition: Any process that stops, prevents or reduces the frequency, rate or extent of endocytic recycling. Relationships: is_a negative regulation of intracellular transport [GO:0032387]; is a type of regulation of endocytic recycling [GO:2001135]; negatively regulates GO:0032456